{
  "gene_name": "Polymeric immunoglobulin receptor",
  "gene": "UniProtKB:P01833",
  "term_label": "signal transduction",
  "gene_symbol": "PIGR",
  "term_id": "GO:0007165"
}